phytochelatin transport [GO:0071993] (BP) Subtypes: phytochelatin transmembrane transport [GO:0071994] Definition: The directed movement of a phytochelatin into, out of or within a cell, or between cells, by means of some agent such as a transporter or pore. Phytochelatins are a group of peptides that bind metals (Cd, Zn, Cu, Pb, Hg) in thiolate coordination complexes. Relationships: is a type of GO:0015711; is a type of amide transport [GO:0042886] Sources: GOC:mah, ISBN:0198506732 Also known as: cadystin transport